{
  "term_id": "GO:0005549",
  "gene_name": "Olfactory receptor 5J2",
  "term_label": "odorant binding",
  "gene_symbol": "OR5J2",
  "gene": "UniProtKB:Q8NH18"
}